{
  "term_label": "Unknown cellular component",
  "gene_name": "Uncharacterized protein",
  "gene": "UniProtKB:A0A2U3TZM8",
  "term_id": "UNKNOWN:0003",
  "gene_symbol": "LOC112694756"
}